regulation of late stripe melanocyte differentiation [GO:0050940] (biological process) Also known as: regulation of late stripe melanophore differentiation Definition: Any process that modulates the frequency, rate or extent of late stripe melanocyte differentiation. Relationships: is a type of regulation of melanocyte differentiation [GO:0045634]; regulates late stripe melanocyte differentiation [GO:0050934] Subtypes: negative regulation of late stripe melanocyte differentiation [GO:0050949], GO:0050950 Sources: GOC:ai